{
  "gene_symbol": "THAP7",
  "gene_name": "THAP domain-containing protein 7",
  "term_label": "regulation of DNA-templated transcription",
  "gene": "UniProtKB:Q9BT49",
  "term_id": "GO:0006355"
}